U5 snRNP [GO:0005682] (cellular component) Sources: GOC:krc, GOC:mah, ISBN:0879695897 Relationships: is a type of spliceosomal snRNP complex [GO:0097525] Definition: A ribonucleoprotein complex that contains small nuclear RNA U5, a heptameric ring of Sm proteins, as well as several proteins that are unique to the U5 snRNP, most of which remain associated with the U5 snRNA both while the U5 snRNP is free or assembled into a series of spliceosomal complexes. Also known as: snRNP U5